{
  "gene_symbol": "EGFL7",
  "gene": "UniProtKB:Q9UHF1",
  "gene_name": "Epidermal growth factor-like protein 7",
  "term_id": "GO:0009986",
  "term_label": "cell surface"
}